{
  "gene": "UniProtKB:Q14671",
  "term_label": "miRNA processing",
  "gene_symbol": "PUM1",
  "gene_name": "Pumilio homolog 1",
  "term_id": "GO:0035196"
}